{
  "term_label": "plasma membrane",
  "gene": "UniProtKB:Q9H427",
  "gene_name": "Potassium channel subfamily K member 15",
  "term_id": "GO:0005886",
  "gene_symbol": "KCNK15"
}